{
  "gene": "UniProtKB:Q05066",
  "term_label": "nucleus",
  "term_id": "GO:0005634",
  "gene_symbol": "SRY",
  "gene_name": "Sex-determining region Y protein"
}